shikimate kinase activity [GO:0004765] (molecular function) Also known as: ATP:shikimate 3-phosphotransferase activity, shikimate kinase (phosphorylating), shikimate kinase II Definition: Catalysis of the reaction: ATP + shikimate = 3-phosphoshikimate + ADP + 2 H+. Sources: EC:2.7.1.71, RHEA:13121 Relationships: is a type of kinase activity [GO:0016301]; is a type of phosphotransferase activity, alcohol group as acceptor [GO:0016773]